{
  "gene": "UniProtKB:P05198",
  "gene_name": "Eukaryotic translation initiation factor 2 subunit 1",
  "gene_symbol": "EIF2S1",
  "term_label": "translational initiation",
  "term_id": "GO:0006413"
}